{
  "gene": "UniProtKB:Q2M5E4",
  "term_id": "GO:0009898",
  "gene_name": "Regulator of G-protein signaling 21",
  "gene_symbol": "RGS21",
  "term_label": "cytoplasmic side of plasma membrane"
}